negative regulation of deadenylation-dependent decapping of nuclear-transcribed mRNA [GO:0106289] (biological process) Relationships: is a type of regulation of deadenylation-dependent decapping of nuclear-transcribed mRNA [GO:0106288]; is a type of GO:1902373; negatively regulates deadenylation-dependent decapping of nuclear-transcribed mRNA [GO:0000290] Definition: Any process that stops, prevents, or reduces the frequency, rate or extent of deadenylation-dependent decapping of nuclear-transcribed mRNA. References: PMID:32354837